positive regulation of ubiquitin-dependent protein catabolic process [GO:2000060] (biological process) Also known as: positive regulation of protein ubiquitination during ubiquitin-dependent protein breakdown, positive regulation of protein ubiquitination during ubiquitin-dependent protein catabolism, positive regulation of protein ubiquitination during ubiquitin-dependent protein degradation, positive regulation of protein ubiquitination involved in ubiquitin-dependent protein catabolic process, positive regulation of protein ubiquitinylation during ubiquitin-dependent protein catabolic process, positive regulation of protein ubiquitinylation during ubiquitin-dependent protein catabolism, positive regulation of protein ubiquitylation during ubiquitin-dependent protein catabolic process, positive regulation of protein ubiquitylation during ubiquitin-dependent protein catabolism, positive regulation of protein degradation tagging activity Sources: GOC:BHF Subtypes: positive regulation of proteasomal ubiquitin-dependent protein catabolic process [GO:0032436] Relationships: is a type of positive regulation of catabolic process [GO:0009896]; is a type of positive regulation of proteolysis involved in protein catabolic process [GO:1903052]; is a type of regulation of ubiquitin-dependent protein catabolic process [GO:2000058]; positively regulates ubiquitin-dependent protein catabolic process [GO:0006511] Definition: Any process that activates or increases the frequency, rate or extent of ubiquitin-dependent protein catabolic process.